{
  "term_label": "Unknown molecular function",
  "gene_symbol": "MICA",
  "gene_name": "MHC class I polypeptide-related sequence A",
  "gene": "UniProtKB:Q29983",
  "term_id": "UNKNOWN:0001"
}